{
  "term_id": "GO:0007265",
  "gene_symbol": "RASGRP1",
  "term_label": "Ras protein signal transduction",
  "gene_name": "RAS guanyl-releasing protein 1",
  "gene": "UniProtKB:O95267"
}